chondrocyte morphogenesis [GO:0090171] (biological process) Relationships: is a type of GO:0000902; is part of chondrocyte development [GO:0002063] Definition: The process in which the structures of a chondrocyte are generated and organized. This process occurs while the initially relatively unspecialized cell is acquiring the specialized features of a chondrocyte. Sources: GOC:ascb_2009, GOC:dph, GOC:tb Subtypes: chondrocyte morphogenesis involved in endochondral bone morphogenesis [GO:0003414]